gene silencing by piRNA-directed DNA methylation [GO:0141176] (biological process) References: PMID:32674113, PMID:38359823 Definition: A small RNA-based gene silencing process in which Piwi-associated RNAs (piRNAs) guide de novo DNA methylation. This results in a heterochromatin assembly, a chromatin conformation that is refractory to transcription. Relationships: is_a GO:0006346; is a type of piRNA-mediated heterochromatin formation [GO:0140966] Subtypes: transposable element silencing by piRNA-mediated DNA methylation [GO:0141196]